plus-end-directed endosome transport along mitotic spindle midzone microtubule [GO:0140024] (biological process) References: PMID:24803650, PMID:25706234 Relationships: is a type of GO:0072383 Definition: The directed movement of an endosome towards the plus end of a microtubule, mediated by motor proteins. This process begins with the attachment of an endosome to a microtubule, and ends when the endosome reaches its final destination.